symmetric, GABA-ergic, inhibitory synapse [GO:0098983] (cellular component) Relationships: is a type of symmetric synapse [GO:0032280]; is_a inhibitory synapse [GO:0060077]; is a type of GABA-ergic synapse [GO:0098982] Definition: A neuron to neuron synapse that lacks an electron dense postsynaptic specialization, uses GABA as a neurotransmitter and whose activity results in inhibitory postsynaptic potentials. Sources: GOC:dos